{
  "gene": "UniProtKB:O75461",
  "term_id": "GO:0090575",
  "gene_name": "Transcription factor E2F6",
  "term_label": "RNA polymerase II transcription regulator complex",
  "gene_symbol": "E2F6"
}